ommochrome biosynthetic process [GO:0006727] (biological process) Sources: ISBN:0198506732 Also known as: ommochrome anabolism, ommochrome biosynthesis, ommochrome formation, ommochrome synthesis Relationships: is a type of eye pigment biosynthetic process [GO:0006726]; is a type of ocellus pigment biosynthetic process [GO:0008055]; is a type of ommochrome metabolic process [GO:0046152] Definition: The chemical reactions and pathways resulting in the formation of ommochromes, any of a large group of natural polycyclic pigments commonly found in the Arthropoda, particularly in the ommatidia of the compound eye.